{
  "term_label": "chloride transmembrane transport",
  "gene_symbol": "GABRB1",
  "gene": "UniProtKB:P18505",
  "gene_name": "Gamma-aminobutyric acid receptor subunit beta-1",
  "term_id": "GO:1902476"
}